{
  "gene_name": "ETS-related transcription factor Elf-4",
  "term_label": "nucleus",
  "term_id": "GO:0005634",
  "gene_symbol": "ELF4",
  "gene": "UniProtKB:Q99607"
}